(+)-lariciresinol catabolic process [GO:1902131] (biological process) Also known as: (+)-lariciresinol breakdown, (+)-lariciresinol catabolism, (+)-lariciresinol degradation Definition: The chemical reactions and pathways resulting in the breakdown of (+)-lariciresinol. Relationships: is a type of phenol-containing compound catabolic process [GO:0019336]; is a type of primary alcohol catabolic process [GO:0034310]; is_a lignan catabolic process [GO:0046273]; is a type of ether catabolic process [GO:1901502] References: PMID:8910615, PMID:9872995 Sources: GOC:TermGenie